{
  "term_label": "Golgi organization",
  "gene_symbol": "TMED9",
  "gene_name": "Transmembrane emp24 domain-containing protein 9",
  "gene": "UniProtKB:Q9BVK6",
  "term_id": "GO:0007030"
}